{
  "gene_symbol": "ITPR1",
  "term_id": "GO:0005220",
  "gene": "UniProtKB:Q14643",
  "gene_name": "Inositol 1,4,5-trisphosphate receptor type 1",
  "term_label": "inositol 1,4,5-trisphosphate-gated calcium channel activity"
}